{
  "gene": "UniProtKB:Q2M1K9",
  "gene_symbol": "ZNF423",
  "gene_name": "Zinc finger protein 423",
  "term_id": "GO:0000978",
  "term_label": "RNA polymerase II cis-regulatory region sequence-specific DNA binding"
}